{
  "term_id": "GO:0005829",
  "gene_name": "Guanine nucleotide exchange factor subunit RIC1",
  "gene_symbol": "RIC1",
  "gene": "UniProtKB:Q4ADV7",
  "term_label": "cytosol"
}